regulation of motile cilium assembly [GO:1905503] (biological process) Definition: Any process that modulates the frequency, rate or extent of motile cilium assembly. References: PMID:25294941 Sources: GOC:TermGenie, GOC:cilia, GOC:krc, GO_REF:0000058 Also known as: regulation of motile primary cilia assembly, regulation of motile primary cilia formation, regulation of motile primary cilium assembly, regulation of motile primary cilium formation, regulation of nodal cilium assembly, regulation of nodal cilium formation Relationships: is_a GO:1902017; regulates GO:0044458 Subtypes: negative regulation of motile cilium assembly [GO:1905504], positive regulation of motile cilium assembly [GO:1905505]